negative regulation of intestinal cholesterol absorption [GO:0045796] (biological process) Definition: Any process that stops, prevents, or reduces the frequency, rate or extent of uptake of cholesterol into the blood by absorption from the intestine. Sources: GOC:go_curators Also known as: down regulation of cholesterol absorption, down-regulation of cholesterol absorption, downregulation of cholesterol absorption, inhibition of cholesterol absorption Relationships: is a type of regulation of intestinal cholesterol absorption [GO:0030300]; is a type of negative regulation of intestinal lipid absorption [GO:1904730]; negatively regulates intestinal cholesterol absorption [GO:0030299]